{
  "gene_name": "Synaptic vesicular amine transporter",
  "term_label": "aminergic neurotransmitter loading into synaptic vesicle",
  "gene": "UniProtKB:Q05940",
  "gene_symbol": "SLC18A2",
  "term_id": "GO:0015842"
}